{
  "term_id": "GO:0007155",
  "gene_symbol": "PARD3B",
  "gene": "UniProtKB:Q8TEW8",
  "gene_name": "Partitioning defective 3 homolog B",
  "term_label": "cell adhesion"
}